{
  "gene_symbol": "POU5F1B",
  "term_label": "RNA polymerase II cis-regulatory region sequence-specific DNA binding",
  "term_id": "GO:0000978",
  "gene_name": "Putative POU domain, class 5, transcription factor 1B",
  "gene": "UniProtKB:Q06416"
}